{
  "term_id": "GO:0005634",
  "gene": "UniProtKB:Q6ZN11",
  "gene_symbol": "ZNF793",
  "gene_name": "Zinc finger protein 793",
  "term_label": "nucleus"
}